{
  "term_id": "GO:0007155",
  "gene_name": "Folate receptor beta",
  "gene": "UniProtKB:P14207",
  "term_label": "cell adhesion",
  "gene_symbol": "FOLR2"
}